{
  "gene": "UniProtKB:O75190",
  "term_label": "protein folding",
  "gene_symbol": "DNAJB6",
  "term_id": "GO:0006457",
  "gene_name": "DnaJ homolog subfamily B member 6"
}